{
  "gene": "UniProtKB:O75154",
  "gene_name": "Rab11 family-interacting protein 3",
  "term_label": "endocytic recycling",
  "gene_symbol": "RAB11FIP3",
  "term_id": "GO:0032456"
}